{
  "gene": "UniProtKB:O75191",
  "gene_name": "Xylulose kinase",
  "term_label": "xylulose metabolic process",
  "gene_symbol": "XYLB",
  "term_id": "GO:0005997"
}